regulation of axial mesodermal cell fate specification [GO:0048328] (biological process) Subtypes: GO:0048329, positive regulation of axial mesodermal cell fate specification [GO:0048330] Relationships: is a type of regulation of mesodermal cell fate specification [GO:0042661]; regulates axial mesodermal cell fate specification [GO:0048327] Definition: Any process that modulates the frequency, rate or extent of axial mesoderm cell fate specification. Sources: GOC:dgh